{
  "gene": "UniProtKB:Q8NH90",
  "gene_name": "Olfactory receptor 5AK2",
  "term_id": "UNKNOWN:0003",
  "term_label": "Unknown cellular component",
  "gene_symbol": "OR5AK2"
}